{
  "gene_symbol": "AHSP",
  "term_id": "GO:0050821",
  "term_label": "protein stabilization",
  "gene_name": "Alpha-hemoglobin-stabilizing protein",
  "gene": "UniProtKB:Q9NZD4"
}